{
  "term_label": "regulation of transcription by RNA polymerase II",
  "gene_name": "CDK-activating kinase assembly factor MAT1",
  "term_id": "GO:0006357",
  "gene": "UniProtKB:P51948",
  "gene_symbol": "MNAT1"
}